{
  "gene_name": "DNA dC-dU-editing enzyme APOBEC-3B",
  "term_id": "GO:0003723",
  "gene_symbol": "APOBEC3B",
  "gene": "UniProtKB:Q9UH17",
  "term_label": "RNA binding"
}